clathrin-dependent endocytosis [GO:0072583] (biological process) Definition: An endocytosis process that begins when material is taken up into clathrin-coated pits, which then pinch off to form clathrin-coated endocytic vesicles. Regulation: negatively regulated by negative regulation of clathrin-dependent endocytosis [GO:1900186]; regulated by regulation of clathrin-dependent endocytosis [GO:2000369]; positively regulated by GO:2000370 Relationships: is_a receptor-mediated endocytosis [GO:0006898] Subtypes: clathrin-dependent endocytosis involved in vitellogenesis [GO:0061883], clathrin-dependent endocytosis of virus by host cell [GO:0075512], clathrin-dependent synaptic vesicle endocytosis [GO:0150007], clathrin-dependent extracellular exosome endocytosis [GO:1990771] References: PMID:18498251, PMID:8970738, PMID:9234965 Sources: GOC:BHF, GOC:mah Also known as: CME, clathrin coated pit-dependent endocytosis, clathrin-mediated endocytosis